chlorophyllide a oxygenase activity [GO:0010277] (molecular function) Definition: Catalysis of the reactions: chlorophyllide a + 2 H+ + 2 NADPH + 2 O2 = chlorophyllide b + 3 H2O + 2 NADP+. Sources: RHEA:30359 Also known as: CAO activity, chlorophyll a oxygenation activity, chlorophyll b synthesis activity, chlorophyll-b synthesis activity, chlorophyllide a:oxygen 7-oxidoreduction activity, chlorophyllide-a oxygenation activity Relationships: is a type of oxidoreductase activity, acting on single donors with incorporation of molecular oxygen, incorporation of one atom of oxygen (internal monooxygenases or internal mixed function oxidases) [GO:0016703]